{
  "gene_name": "18S rRNA aminocarboxypropyltransferase",
  "term_label": "Unknown molecular function",
  "term_id": "UNKNOWN:0001",
  "gene": "UniProtKB:Q9UJK0",
  "gene_symbol": "TSR3"
}